{
  "gene_name": "Immunoglobulin kappa joining 4 (Fragment)",
  "term_id": "UNKNOWN:0002",
  "term_label": "Unknown biological process",
  "gene": "UniProtKB:A0A0A0MT69",
  "gene_symbol": "IGKJ4"
}